{
  "gene": "UniProtKB:P48745",
  "gene_name": "CCN family member 3",
  "gene_symbol": "CCN3",
  "term_id": "GO:0002062",
  "term_label": "chondrocyte differentiation"
}